{
  "gene_symbol": "FBLN2",
  "term_label": "extracellular matrix binding",
  "gene_name": "Fibulin-2",
  "gene": "UniProtKB:P98095",
  "term_id": "GO:0050840"
}